{
  "term_id": "GO:0008292",
  "term_label": "acetylcholine biosynthetic process",
  "gene_name": "Choline O-acetyltransferase",
  "gene": "UniProtKB:P28329",
  "gene_symbol": "CHAT"
}